{
  "term_label": "protein-DNA covalent cross-linking repair",
  "gene_symbol": "TEX264",
  "gene": "UniProtKB:Q9Y6I9",
  "term_id": "GO:0106300",
  "gene_name": "Testis-expressed protein 264"
}